negative regulation of signal transduction [GO:0009968] (biological process) Definition: Any process that stops, prevents, or reduces the frequency, rate or extent of signal transduction. Subtypes: negative regulation of cytokine-mediated signaling pathway [GO:0001960], negative regulation of abscisic acid-activated signaling pathway [GO:0009788], negative regulation of gibberellic acid mediated signaling pathway [GO:0009938], negative regulation of platelet-derived growth factor receptor signaling pathway [GO:0010642], GO:0010754, negative regulation of auxin mediated signaling pathway [GO:0010930], negative adaptation of signaling pathway [GO:0022401], termination of signal transduction [GO:0023021], GO:0030178, negative regulation of vascular endothelial growth factor receptor signaling pathway [GO:0030948], negative regulation of brain-derived neurotrophic factor receptor signaling pathway [GO:0031549], GO:0031665, negative regulation of toll-like receptor signaling pathway [GO:0034122], GO:0034132, negative regulation of toll-like receptor 2 signaling pathway [GO:0034136], negative regulation of toll-like receptor 4 signaling pathway [GO:0034144], negative regulation of toll-like receptor 5 signaling pathway [GO:0034148], GO:0034152, GO:0034168, GO:0035387, GO:0038011, negative regulation of fibroblast growth factor receptor signaling pathway [GO:0040037], negative regulation of insulin-like growth factor receptor signaling pathway [GO:0043569], GO:0045744, negative regulation of Notch signaling pathway [GO:0045746], negative regulation of Toll signaling pathway [GO:0045751], negative regulation of sevenless signaling pathway [GO:0045873], negative regulation of smoothened signaling pathway [GO:0045879], negative regulation of insulin receptor signaling pathway [GO:0046627], negative regulation of antigen receptor-mediated signaling pathway [GO:0050858], negative regulation of neurotrophin TRK receptor signaling pathway [GO:0051387], negative regulation of signal transduction involved in conjugation with cellular fusion [GO:0060240], negative regulation of cytokine activity [GO:0060302], negative regulation of growth hormone receptor signaling pathway [GO:0060400], GO:0061060, negative regulation of cytokinin-activated signaling pathway [GO:0080037], negative regulation of transmembrane receptor protein serine/threonine kinase signaling pathway [GO:0090101], negative regulation of red or far-red light signaling pathway [GO:0090229], negative regulation of torso signaling pathway [GO:0120177], negative regulation of GDF15-GFRAL signaling pathway [GO:0160145], negative regulation of corticotropin-releasing hormone receptor activity [GO:1900011], extracellular negative regulation of signal transduction [GO:1900116], GO:1900450, negative regulation of brassinosteroid mediated signaling pathway [GO:1900458], negative regulation of vascular endothelial growth factor signaling pathway [GO:1900747], negative regulation of signal transduction in absence of ligand [GO:1901099], negative regulation of ERBB signaling pathway [GO:1901185], negative regulation of ephrin receptor signaling pathway [GO:1901188], negative regulation of Fas signaling pathway [GO:1902045], negative regulation of sphingolipid mediated signaling pathway [GO:1902069], negative regulation of hepatocyte growth factor receptor signaling pathway [GO:1902203], negative regulation of intracellular signal transduction [GO:1902532], negative regulation of glucose mediated signaling pathway [GO:1902660], GO:1902842, GO:1902848, GO:1904893, negative regulation of apolipoprotein A-I-mediated signaling pathway [GO:1905095], negative regulation of Fc-gamma receptor signaling pathway involved in phagocytosis [GO:1905450], GO:2000349, GO:2000441, negative regulation of glial cell-derived neurotrophic factor receptor signaling pathway involved in ureteric bud formation [GO:2000734], GO:2001045, negative regulation of apoptotic signaling pathway [GO:2001234], GO:2001261 Sources: GOC:sm Relationships: is a type of regulation of signal transduction [GO:0009966]; is a type of negative regulation of cell communication [GO:0010648]; is a type of GO:0023057; is a type of GO:0048585; negatively regulates signal transduction [GO:0007165] Also known as: down regulation of signal transduction, down-regulation of signal transduction, downregulation of signal transduction, inhibition of signal transduction, negative regulation of signaling pathway, negative regulation of signalling pathway